{
  "gene_name": "Lymphoid enhancer-binding factor 1",
  "gene_symbol": "LEF1",
  "gene": "UniProtKB:Q9UJU2",
  "term_label": "chromatin",
  "term_id": "GO:0000785"
}